{
  "gene": "UniProtKB:Q96DX4",
  "gene_name": "RING finger and SPRY domain-containing protein 1",
  "gene_symbol": "RSPRY1",
  "term_label": "ubiquitin-protein transferase activity",
  "term_id": "GO:0004842"
}